{
  "gene": "UniProtKB:Q86YL7",
  "term_label": "apical plasma membrane",
  "gene_symbol": "PDPN",
  "term_id": "GO:0016324",
  "gene_name": "Podoplanin"
}